phyllotactic patterning [GO:0060771] (biological process) Subtypes: leaf phyllotactic patterning [GO:0060772], flower phyllotactic patterning [GO:0060773], inflorescence phyllotactic patterning [GO:0090643] Definition: The radial pattern formation process that results in the formation of plant organs (leaves or leaf-like structures) or flower primordia around a central axis. Relationships: is a type of radial pattern formation [GO:0009956] Sources: GOC:dph, GOC:sdb_2009, GOC:tb